{
  "gene": "UniProtKB:P13521",
  "gene_symbol": "SCG2",
  "gene_name": "Secretogranin-2",
  "term_id": "GO:0001525",
  "term_label": "angiogenesis"
}